establishment of tissue polarity [GO:0007164] (biological process) Sources: GOC:jid Subtypes: establishment of planar polarity [GO:0001736] Relationships: is a type of GO:0009653 Definition: Coordinated organization of groups of cells in a tissue, such that they all orient to similar coordinates.